cellular response to purine-containing compound [GO:0071415] (biological process) Definition: Any process that results in a change in state or activity of a cell (in terms of movement, secretion, enzyme production, gene expression, etc.) as a result of a purine-containing compound stimulus. Relationships: is a type of GO:0014074 Sources: GOC:mah Also known as: cellular response to purine Subtypes: cellular response to caffeine [GO:0071313], cellular response to purvalanol A [GO:0072754], GO:0072764